{
  "gene": "UniProtKB:Q8TAM6",
  "term_label": "internode region of axon",
  "gene_name": "Ermin",
  "term_id": "GO:0033269",
  "gene_symbol": "ERMN"
}